active sex chromosome [GO:0098579] (cellular component) Definition: A sex chromosome that has not been inactivated. Sources: GOC:dos Relationships: is a type of sex chromosome [GO:0000803]